{
  "term_id": "GO:0006879",
  "gene": "UniProtKB:P48200",
  "gene_name": "Iron-responsive element-binding protein 2",
  "term_label": "intracellular iron ion homeostasis",
  "gene_symbol": "IREB2"
}